hydroxymethylglutaryl-CoA lyase activity [GO:0004419] (molecular function) Relationships: is a type of GO:0016833 Sources: EC:4.1.3.4, RHEA:24404 Definition: Catalysis of the reaction: (S)-3-hydroxy-3-methylglutaryl-CoA = acetoacetate + acetyl-CoA. Also known as: (S)-3-hydroxy-3-methylglutaryl-CoA acetoacetate-lyase (acetyl-CoA-forming), (S)-3-hydroxy-3-methylglutaryl-CoA acetoacetate-lyase activity, 3-hydroxy-3-methylglutarate-CoA lyase activity, 3-hydroxy-3-methylglutaryl CoA cleaving enzyme, 3-hydroxy-3-methylglutaryl coenzyme A lyase activity, 3-hydroxy-3-methylglutaryl-CoA lyase activity, HMG-CoA lyase activity, hydroxymethylglutaryl coenzyme A lyase activity, hydroxymethylglutaryl coenzyme A-cleaving enzyme